{
  "term_label": "NuRD complex",
  "gene_symbol": "GATAD2A",
  "term_id": "GO:0016581",
  "gene_name": "Transcriptional repressor p66-alpha",
  "gene": "UniProtKB:Q86YP4"
}